photoreceptor cell cilium [GO:0097733] (cellular component) Sources: GOC:cilia, Wikipedia:Photoreceptor_cell#Histology Relationships: is_a neuron projection [GO:0043005]; is a type of 9+0 non-motile cilium [GO:0097731] Definition: A specialised 9+0 non-motile cilium found in photoreceptor cells. A ciliary transition zone called 'photoreceptor connecting cilium' links the photoreceptor outer segment to the inner segment. Also known as: photoreceptor cilium